phosphatidylcholine 12-monooxygenase activity [GO:0050183] (molecular function) Also known as: oleate D12-hydroxylase activity, 1-acyl-2-oleoyl-sn-glycero-3-phosphocholine,NADH:oxygen oxidoreductase (12-hydroxylating), oleate Delta(12)-hydroxylase activity, oleate delta12-hydroxylase activity, oleate delta12-monooxygenase activity, ricinoleic acid synthase activity Definition: Catalysis of the reaction: 1-acyl-2-(9Z)-octadecenoyl-sn-glycero-3-phosphocholine + 2 Fe(II)-[cytochrome b5] + 2 H+ + O2 = 1-acyl-2-[(R)-12-hydroxyoleoyl]-sn-glycero-3-phosphocholine + 2 Fe(III)-[cytochrome b5] + H2O. Relationships: is a type of oxidoreductase activity, acting on paired donors, with incorporation or reduction of molecular oxygen, another compound as one donor, and incorporation of one atom of oxygen [GO:0016716] Sources: RHEA:46360